negative regulation of TOR signaling [GO:0032007] (biological process) Subtypes: GO:1903940, GO:1904262 Also known as: down regulation of TOR signaling pathway, down-regulation of TOR signaling pathway, downregulation of TOR signaling pathway, negative regulation of TOR signaling pathway, negative regulation of TOR signalling pathway, negative regulation of target of rapamycin signaling pathway, negative regulation of target of rapamycin signalling pathway, inhibition of TOR signaling pathway, negative regulation of TOR signaling cascade Definition: Any process that stops, prevents, or reduces the frequency, rate or extent of TOR signaling. Sources: GOC:mah Relationships: is a type of GO:0032006; is a type of negative regulation of intracellular signal transduction [GO:1902532]; negatively regulates GO:0031929